{
  "term_id": "GO:0005874",
  "term_label": "microtubule",
  "gene": "UniProtKB:Q6PEY2",
  "gene_symbol": "TUBA3E",
  "gene_name": "Tubulin alpha-3E chain"
}